{
  "gene": "UniProtKB:O95758",
  "gene_name": "Polypyrimidine tract-binding protein 3",
  "gene_symbol": "PTBP3",
  "term_id": "GO:0043484",
  "term_label": "regulation of RNA splicing"
}